{
  "term_label": "regulation of neuroblast proliferation",
  "gene": "UniProtKB:Q7Z5A9",
  "gene_name": "Chemokine-like protein TAFA-1",
  "gene_symbol": "TAFA1",
  "term_id": "GO:1902692"
}